{
  "gene_name": "Sodium_potassium-transporting ATPase subunit alpha-3",
  "term_label": "sodium ion export across plasma membrane",
  "term_id": "GO:0036376",
  "gene": "UniProtKB:P13637",
  "gene_symbol": "ATP1A3"
}